{
  "gene": "UniProtKB:P49321",
  "gene_symbol": "NASP",
  "term_label": "nucleoplasm",
  "term_id": "GO:0005654",
  "gene_name": "Nuclear autoantigenic sperm protein"
}